{
  "gene": "UniProtKB:Q96P69",
  "gene_symbol": "GPR78",
  "term_id": "GO:0004930",
  "gene_name": "G-protein coupled receptor 78",
  "term_label": "G protein-coupled receptor activity"
}